{
  "term_id": "UNKNOWN:0003",
  "gene_symbol": "COL26A1",
  "gene": "UniProtKB:Q96A83",
  "term_label": "Unknown cellular component",
  "gene_name": "Collagen alpha-1(XXVI) chain"
}